{
  "gene_symbol": "PCDHA12",
  "gene": "UniProtKB:Q9UN75",
  "gene_name": "Protocadherin alpha-12",
  "term_label": "plasma membrane",
  "term_id": "GO:0005886"
}